voltage-gated calcium channel activity involved in regulation of postsynaptic cytosolic calcium levels [GO:1905057] (molecular function) Definition: Any voltage-gated calcium channel activity that is involved in regulation of postsynaptic cytosolic calcium ion concentration. Relationships: is a type of voltage-gated calcium channel activity involved in regulation of cytosolic calcium levels [GO:0099511]; is part of GO:0099566 Also known as: depolarization-activated voltage gated calcium channel activity involved in regulation of postsynaptic cytosolic calcium ion concentration, depolarization-activated voltage-gated calcium channel activity involved in regulation of postsynaptic cytosolic calcium ion concentration, depolarization-activated voltage-gated calcium channel involved in regulation of postsynaptic cytosolic calcium ion concentration, voltage gated calcium channel activity involved in regulation of postsynaptic cytosolic calcium ion concentration, voltage-dependent calcium channel activity involved in regulation of postsynaptic cytosolic calcium ion concentration, voltage-gated calcium channel activity involved in regulation of postsynaptic cytosolic calcium levels, voltage-gated calcium ion channel activity involved in regulation of postsynaptic cytosolic calcium ion concentration, voltage-sensitive calcium channel involved in regulation of postsynaptic cytosolic calcium ion concentration, dihydropyridine-sensitive calcium channel activity involved in regulation of postsynaptic cytosolic calcium ion concentration References: PMID:20734177 Sources: GOC:TermGenie, GO_REF:0000061